{
  "term_id": "GO:0000981",
  "gene": "UniProtKB:P20264",
  "gene_name": "POU domain, class 3, transcription factor 3",
  "term_label": "DNA-binding transcription factor activity, RNA polymerase II-specific",
  "gene_symbol": "POU3F3"
}